{
  "term_label": "lipid binding",
  "gene_symbol": "APOL5",
  "gene_name": "Apolipoprotein L5",
  "gene": "UniProtKB:Q9BWW9",
  "term_id": "GO:0008289"
}